{
  "gene": "UniProtKB:O43612",
  "gene_name": "Hypocretin neuropeptide precursor",
  "term_id": "GO:0042755",
  "term_label": "eating behavior",
  "gene_symbol": "HCRT"
}